response to type I interferon [GO:0034340] (biological process) Subtypes: cellular response to type I interferon [GO:0071357] Definition: Any process that results in a change in state or activity of a cell or an organism (in terms of movement, secretion, enzyme production, gene expression, etc.) as a result of a type I interferon stimulus. Type I interferons include the interferon-alpha, beta, delta, episilon, zeta, kappa, tau, and omega gene families. Also known as: response to type I IFN References: PMID:15546383, PMID:16681834 Sources: GOC:add, ISBN:0126896631 Relationships: is a type of response to cytokine [GO:0034097]; is part of innate immune response [GO:0045087]